{
  "gene": "UniProtKB:Q03431",
  "gene_symbol": "PTH1R",
  "gene_name": "Parathyroid hormone_parathyroid hormone-related peptide receptor",
  "term_label": "parathyroid hormone receptor activity",
  "term_id": "GO:0004991"
}